{
  "gene_name": "Deubiquitinating protein VCPIP1",
  "gene": "UniProtKB:Q96JH7",
  "term_label": "protein-DNA covalent cross-linking repair",
  "term_id": "GO:0106300",
  "gene_symbol": "VCPIP1"
}